{
  "term_id": "GO:0019814",
  "gene_symbol": "IGKV1OR2-108",
  "term_label": "immunoglobulin complex",
  "gene": "UniProtKB:A0A075B7D4",
  "gene_name": "Immunoglobulin kappa variable 1_OR2-108 (non-functional) (Fragment)"
}